{
  "gene_symbol": "MEIS2",
  "term_id": "GO:0009887",
  "gene_name": "Homeobox protein Meis2",
  "term_label": "animal organ morphogenesis",
  "gene": "UniProtKB:O14770"
}